cellular response to hydroxyisoflavone [GO:0071413] (BP) Definition: Any process that results in a change in state or activity of a cell (in terms of movement, secretion, enzyme production, gene expression, etc.) as a result of a hydroxyisoflavone stimulus. Relationships: is a type of response to hydroxyisoflavone [GO:0033594]; is a type of cellular response to ketone [GO:1901655]; is a type of cellular response to phenylpropanoid [GO:1905546] Subtypes: cellular response to genistein [GO:0071412] Sources: GOC:mah